{
  "gene_symbol": "TMEM98",
  "term_label": "endoplasmic reticulum",
  "gene": "UniProtKB:Q9Y2Y6",
  "gene_name": "Transmembrane protein 98",
  "term_id": "GO:0005783"
}